{
  "gene": "UniProtKB:P42568",
  "term_label": "transcription elongation factor complex",
  "gene_symbol": "MLLT3",
  "term_id": "GO:0008023",
  "gene_name": "Protein AF-9"
}